{
  "term_id": "GO:0003682",
  "gene": "UniProtKB:O43918",
  "gene_name": "Autoimmune regulator",
  "gene_symbol": "AIRE",
  "term_label": "chromatin binding"
}